{
  "gene_symbol": "KCTD11",
  "gene": "UniProtKB:Q693B1",
  "gene_name": "BTB_POZ domain-containing protein KCTD11",
  "term_label": "Unknown molecular function",
  "term_id": "UNKNOWN:0001"
}